PYM-mago-Y14 complex [GO:1990509] (cellular component) Note: An example of this is wibg in Drosophila melanogaster (P82804) in PMID:14968132 (inferred from physical interaction). References: PMID:14968132 Sources: GOC:bhm Also known as: PYM-mago-RNA-binding protein 8A complex, wibg-mago-tsu complex Relationships: is a type of protein-containing complex [GO:0032991]; has part exon-exon junction subcomplex mago-y14 [GO:1990501] Definition: Protein complex involved in the disassembly of Mago-Y14 from the spliced mRNA during first round of translation, independently of the translational machinery. Conserved from fission yeast to humans.